{
  "gene": "UniProtKB:Q9NNX6",
  "term_id": "GO:0009897",
  "gene_name": "CD209 antigen",
  "term_label": "external side of plasma membrane",
  "gene_symbol": "CD209"
}